{
  "gene": "UniProtKB:Q9Y274",
  "gene_symbol": "ST3GAL6",
  "term_label": "Unknown cellular component",
  "gene_name": "Type 2 lactosamine alpha-2,3-sialyltransferase",
  "term_id": "UNKNOWN:0003"
}